{
  "term_label": "DNA-directed RNA polymerase activity",
  "gene_name": "DNA primase small subunit",
  "term_id": "GO:0003899",
  "gene_symbol": "PRIM1",
  "gene": "UniProtKB:P49642"
}